{
  "gene_name": "Coatomer subunit beta",
  "term_id": "GO:0030126",
  "term_label": "COPI vesicle coat",
  "gene": "UniProtKB:P53618",
  "gene_symbol": "COPB1"
}